{
  "gene_symbol": "TMEM210",
  "term_label": "Unknown molecular function",
  "gene": "UniProtKB:A6NLX4",
  "gene_name": "Transmembrane protein 210",
  "term_id": "UNKNOWN:0001"
}